{
  "gene": "UniProtKB:Q99943",
  "gene_name": "1-acyl-sn-glycerol-3-phosphate acyltransferase alpha",
  "term_label": "endoplasmic reticulum",
  "gene_symbol": "AGPAT1",
  "term_id": "GO:0005783"
}